negative regulation of chitin-based cuticle tanning [GO:0045800] (biological process) Subtypes: negative regulation of adult chitin-containing cuticle pigmentation [GO:0048083] Relationships: is a type of regulation of chitin-based cuticle tanning [GO:0007564]; is a type of negative regulation of developmental process [GO:0051093]; is a type of negative regulation of multicellular organismal process [GO:0051241]; negatively regulates chitin-based cuticle sclerotization [GO:0007593] Sources: GOC:go_curators, GOC:jid, GOC:mtg_sensu Definition: Any process that stops, prevents, or reduces the frequency, rate or extent of chitin-based cuticular tanning. Also known as: down regulation of cuticle tanning, down-regulation of cuticle tanning, downregulation of cuticle tanning, negative regulation of cuticle tanning, inhibition of cuticle tanning, negative regulation of cuticle hardening